regulation of timing of subpallium neuron differentiation [GO:0060165] (biological process) Relationships: is a type of GO:0060164; is part of GO:0021544 Definition: The process controlling the timing and/or rate at which a relatively unspecialized cell in the subpallium acquires features of a neuron. The subpallium is the base region of the telencephalon. Sources: GOC:dph